{
  "term_id": "UNKNOWN:0001",
  "term_label": "Unknown molecular function",
  "gene": "UniProtKB:A0A8I5QKY2",
  "gene_symbol": "A0A8I5QKY2",
  "gene_name": "Uncharacterized protein"
}